{
  "gene": "UniProtKB:P49888",
  "term_label": "cytoplasm",
  "term_id": "GO:0005737",
  "gene_symbol": "SULT1E1",
  "gene_name": "Sulfotransferase 1E1"
}